{
  "term_label": "heme biosynthetic process",
  "gene_symbol": "ALAS2",
  "gene_name": "5-aminolevulinate synthase, erythroid-specific, mitochondrial",
  "gene": "UniProtKB:P22557",
  "term_id": "GO:0006783"
}